{
  "gene_name": "Sterol O-acyltransferase 1",
  "term_label": "endoplasmic reticulum membrane",
  "term_id": "GO:0005789",
  "gene_symbol": "SOAT1",
  "gene": "UniProtKB:P35610"
}